{
  "term_label": "Unknown molecular function",
  "gene_name": "p53-regulated apoptosis-inducing protein 1",
  "gene": "UniProtKB:Q9HCN2",
  "gene_symbol": "TP53AIP1",
  "term_id": "UNKNOWN:0001"
}